oocyte morphogenesis [GO:0048601] (biological process) Sources: GOC:go_curators Relationships: is a type of cell morphogenesis [GO:0000902]; is a type of GO:0003006; is part of oocyte development [GO:0048599] Also known as: oocyte morphogenesis during differentiation Definition: The process in which the structures of an oocyte are generated and organized. This process occurs while the initially relatively unspecialized cell is acquiring the specialized features of an oocyte.